{
  "term_id": "UNKNOWN:0002",
  "term_label": "Unknown biological process",
  "gene_symbol": "NUTM2D",
  "gene": "UniProtKB:Q5VT03",
  "gene_name": "NUT family member 2D"
}